{
  "gene": "UniProtKB:P49023",
  "term_label": "Unknown molecular function",
  "gene_name": "Paxillin",
  "gene_symbol": "PXN",
  "term_id": "UNKNOWN:0001"
}